regulation of mitochondrial translation [GO:0070129] (biological process) Also known as: regulation of mitochondrial protein anabolism, regulation of mitochondrial protein biosynthesis, regulation of mitochondrial protein formation, regulation of mitochondrial protein synthesis Sources: GOC:mah Definition: Any process that modulates the frequency, rate or extent of the chemical reactions and pathways resulting in the formation of proteins by the translation of mRNA in a mitochondrion. Relationships: is a type of regulation of translation [GO:0006417]; is a type of regulation of mitochondrial gene expression [GO:0062125]; regulates GO:0032543 Subtypes: negative regulation of mitochondrial translation [GO:0070130], GO:0070131, regulation of mitochondrial translational initiation [GO:0070132]